{
  "gene_symbol": "PVR",
  "gene_name": "Poliovirus receptor",
  "term_id": "GO:0007156",
  "term_label": "homophilic cell-cell adhesion",
  "gene": "UniProtKB:P15151"
}